negative regulation of neural crest formation [GO:0090301] (biological process) Definition: Any process that decreases the rate, frequency, or extent of neural crest formation. Neural crest formation is the formation of the specialized region of ectoderm between the neural ectoderm (neural plate) and non-neural ectoderm. The neural crest gives rise to the neural crest cells that migrate away from this region as neural tube formation proceeds. Sources: GOC:tb Relationships: is a type of negative regulation of epithelial to mesenchymal transition [GO:0010719]; is a type of regulation of neural crest formation [GO:0090299]; negatively regulates neural crest formation [GO:0014029] Subtypes: GO:1905296